acetaldehyde biosynthetic process [GO:0046186] (biological process) Sources: GOC:ai Definition: The chemical reactions and pathways resulting in the formation of acetaldehyde, a colorless, flammable liquid intermediate in the metabolism of alcohol. Relationships: is a type of acetaldehyde metabolic process [GO:0006117]; is a type of aldehyde biosynthetic process [GO:0046184] Also known as: acetaldehyde anabolism, acetaldehyde biosynthesis, acetaldehyde formation, acetaldehyde synthesis